{
  "gene_name": "DEP domain-containing mTOR-interacting protein",
  "gene_symbol": "DEPTOR",
  "term_label": "plasma membrane",
  "term_id": "GO:0005886",
  "gene": "UniProtKB:Q8TB45"
}